snRNA transcription by RNA polymerase III [GO:0042796] (biological process) Definition: The synthesis of small nuclear RNA (snRNA) from a DNA template by RNA Polymerase III (Pol III), originating at a Pol III promoter. Sources: GOC:jl, ISBN:0321000382 Also known as: snRNA transcription from Pol III promoter, snRNA transcription from RNA polymerase III promoter Relationships: is a type of transcription by RNA polymerase III [GO:0006383]; is a type of GO:0009301